histone H3K56 acetyltransferase activity [GO:0032931] (MF) References: PMID:19056256 Also known as: histone H3-K56 acetyltransferase activity, histone acetylase activity (H3-K56 specific), histone acetyltransferase activity (H3-K56 specific), histone lysine N-acetyltransferase activity (H3-K56 specific) Relationships: is a type of histone H3 acetyltransferase activity [GO:0010484] Note: Comment: Note that the residue position corresponds to the canonical human H3 histone (UniProtKB:P84243); this residue is conserved across all eukaryotes. Residue 1 is the first residue following removal of the initiating Methionine (Met). Note that each histone is encoded by multiple genes, and sequences may vary across different genes within an organism. Definition: Catalysis of the reaction: acetyl-CoA + histone H3 L-lysine (position 56) = CoA + histone H3 N6-acetyl-L-lysine (position 56).